immunological memory formation process [GO:0090715] (biological process) Subtypes: GO:0002319, GO:0043379 Definition: Any immunological memory process that can contribute to the formation of immunological memory. Relationships: is a type of immunological memory process [GO:0090713] References: PMID:26086132, PMID:26831526 Sources: GOC:add